{
  "gene_name": "Interleukin-17 receptor A",
  "gene_symbol": "IL17RA",
  "term_id": "UNKNOWN:0002",
  "gene": "UniProtKB:Q96F46",
  "term_label": "Unknown biological process"
}